{
  "gene": "UniProtKB:O60216",
  "term_id": "GO:0003682",
  "gene_name": "Double-strand-break repair protein rad21 homolog",
  "gene_symbol": "RAD21",
  "term_label": "chromatin binding"
}